{
  "gene_name": "Gamma-aminobutyric acid receptor subunit epsilon",
  "term_label": "postsynapse",
  "term_id": "GO:0098794",
  "gene": "UniProtKB:P78334",
  "gene_symbol": "GABRE"
}